{
  "gene_name": "Neuronal PAS domain-containing protein 1",
  "term_id": "GO:0000981",
  "term_label": "DNA-binding transcription factor activity, RNA polymerase II-specific",
  "gene": "UniProtKB:Q99742",
  "gene_symbol": "NPAS1"
}